{
  "gene": "UniProtKB:Q1W4C9",
  "term_label": "Unknown biological process",
  "gene_symbol": "SPINK13",
  "gene_name": "Serine protease inhibitor Kazal-type 13",
  "term_id": "UNKNOWN:0002"
}